{
  "term_label": "early endosome",
  "gene_symbol": "TF",
  "gene": "UniProtKB:P02787",
  "gene_name": "Serotransferrin",
  "term_id": "GO:0005769"
}